{
  "term_label": "plasma membrane",
  "gene_name": "Semaphorin-7A",
  "gene": "UniProtKB:O75326",
  "term_id": "GO:0005886",
  "gene_symbol": "SEMA7A"
}